{
  "term_label": "plasma membrane",
  "gene": "UniProtKB:Q8NG04",
  "term_id": "GO:0005886",
  "gene_symbol": "SLC26A10P",
  "gene_name": "Putative solute carrier family 26 member 10P"
}